release of seed from dormancy [GO:0048838] (BP) Definition: The process in which the dormant state is broken in a seed. Dormancy is characterized by a suspension of physiological activity that can be reactivated upon release. Sources: GOC:dph, GOC:jid, GOC:tb, ISBN:9781405139830 Relationships: is a type of seed dormancy process [GO:0010162]; is a type of exit from dormancy [GO:0097438]